{
  "gene_name": "Protein transport protein Sec16A",
  "gene": "UniProtKB:O15027",
  "term_label": "protein localization to endoplasmic reticulum exit site",
  "gene_symbol": "SEC16A",
  "term_id": "GO:0070973"
}